positive regulation of retinoic acid biosynthetic process [GO:1900054] (biological process) Also known as: activation of retinoic acid anabolic process, positive regulation of retinoic acid anabolic process, up regulation of retinoic acid anabolic process, up-regulation of retinoic acid anabolic process, upregulation of retinoic acid anabolic process, activation of retinoic acid biosynthetic process, up regulation of retinoic acid biosynthetic process, up-regulation of retinoic acid biosynthetic process, upregulation of retinoic acid biosynthetic process Relationships: is a type of positive regulation of hormone metabolic process [GO:0032352]; is a type of GO:0046136; is a type of positive regulation of lipid biosynthetic process [GO:0046889]; is a type of GO:1900052; positively regulates GO:0002138 Definition: Any process that activates or increases the frequency, rate or extent of retinoic acid biosynthetic process. Sources: GOC:TermGenie, GOC:yaf